regulation of skeletal muscle contraction by calcium ion signaling [GO:0014722] (BP) Relationships: is_a regulation of skeletal muscle contraction [GO:0014819]; is a type of calcium-mediated signaling [GO:0019722] Sources: GOC:mtg_muscle Subtypes: regulation of skeletal muscle contraction by modulation of calcium ion sensitivity of myofibril [GO:0014723], regulation of skeletal muscle contraction by regulation of release of sequestered calcium ion [GO:0014809] Definition: Any process that modulates the frequency, rate or extent of skeletal muscle contraction by changing the calcium ion signals that trigger contraction. Also known as: regulation of skeletal muscle contraction by calcium ion signalling